{
  "gene_symbol": "OSBPL3",
  "gene": "UniProtKB:Q9H4L5",
  "term_id": "GO:0005829",
  "term_label": "cytosol",
  "gene_name": "Oxysterol-binding protein-related protein 3"
}